{
  "gene_name": "Chromodomain-helicase-DNA-binding protein 5",
  "term_id": "GO:0016581",
  "gene_symbol": "CHD5",
  "gene": "UniProtKB:Q8TDI0",
  "term_label": "NuRD complex"
}